{
  "gene_symbol": "PKLR",
  "gene_name": "Pyruvate kinase PKLR",
  "gene": "UniProtKB:P30613",
  "term_id": "GO:0004743",
  "term_label": "pyruvate kinase activity"
}